{
  "term_id": "GO:0050900",
  "gene_name": "Integrin alpha-6",
  "term_label": "leukocyte migration",
  "gene": "UniProtKB:P23229",
  "gene_symbol": "ITGA6"
}